{
  "gene_symbol": "XG",
  "term_label": "homotypic cell-cell adhesion",
  "gene": "UniProtKB:P55808",
  "gene_name": "Glycoprotein Xg",
  "term_id": "GO:0034109"
}